{
  "term_label": "heme binding",
  "term_id": "GO:0020037",
  "gene_name": "Tryptophan 2,3-dioxygenase",
  "gene_symbol": "TDO2",
  "gene": "UniProtKB:P48775"
}